very long-chain fatty-acyl-CoA metabolic process [GO:0036111] (biological process) Definition: The chemical reactions and pathways involving very long-chain fatty-acyl-CoAs, any derivative of coenzyme A in which the sulfhydryl group is in a thioester linkage with a very long-chain fatty-acyl group. A very long-chain fatty acid has an aliphatic tail containing more than 22 carbons. Note: While there is not universal consensus on the lengths of short-, medium-, long- and very-long-chain fatty acids, the GO uses the definitions in ChEBI (see CHEBI:26666, CHEBI:59554, CHEBI:15904 and CHEBI:27283). Subtypes: GO:0036113 Sources: GOC:pm Also known as: very long-chain fatty acyl CoA metabolic process, very long-chain fatty acyl-CoA metabolism Relationships: is a type of fatty-acyl-CoA metabolic process [GO:0035337]